{
  "term_id": "GO:0005615",
  "term_label": "extracellular space",
  "gene_name": "Fibromodulin",
  "gene": "UniProtKB:Q06828",
  "gene_symbol": "FMOD"
}